regulation of protein localization to cell division site involved in mitotic actomyosin contractile ring assembly [GO:0110082] (biological process) Subtypes: GO:0110083, negative regulation of protein localization to cell division site involved in mitotic actomyosin contractile ring assembly [GO:0110084] References: PMID:29343550 Sources: GOC:vw Relationships: is a type of regulation of protein localization to cell division site [GO:1901900]; regulates protein localization to cell division site involved in mitotic actomyosin contractile ring assembly [GO:1903476] Definition: Any process that modulates the frequency, rate or extent of protein localization to cell division site involved in mitotic actomyosin contractile ring assembly.